{
  "term_id": "UNKNOWN:0002",
  "gene": "UniProtKB:Q3B7I2",
  "term_label": "Unknown biological process",
  "gene_name": "Protein canopy homolog 1",
  "gene_symbol": "CNPY1"
}